{
  "term_id": "GO:0005739",
  "gene_symbol": "GADD45GIP1",
  "gene_name": "Large ribosomal subunit protein mL64",
  "gene": "UniProtKB:Q8TAE8",
  "term_label": "mitochondrion"
}